{
  "term_id": "GO:0005737",
  "gene_name": "E3 ISG15--protein ligase HERC5",
  "gene_symbol": "HERC5",
  "term_label": "cytoplasm",
  "gene": "UniProtKB:Q9UII4"
}